shoot system development [GO:0048367] (biological process) Also known as: shoot development Definition: The process whose specific outcome is the progression of the shoot system over time, from its formation to the mature structure. Regulation: regulated by regulation of shoot system development [GO:0048831] Relationships: is a type of system development [GO:0048731] Subtypes: shoot regeneration [GO:0062210], reproductive shoot system development [GO:0090567] Sources: GOC:go_curators